positive regulation of protein homotetramerization [GO:1901095] (biological process) Sources: GOC:TermGenie, GOC:pm Also known as: positive regulation of protein homotetramer assembly, positive regulation of protein homotetramer biosynthesis, positive regulation of protein homotetramer biosynthetic process, positive regulation of protein homotetramer formation, up regulation of protein homotetramer assembly, up regulation of protein homotetramer biosynthesis, up regulation of protein homotetramer biosynthetic process, up regulation of protein homotetramer formation, up regulation of protein homotetramerization, up-regulation of protein homotetramer assembly, up-regulation of protein homotetramer biosynthesis, up-regulation of protein homotetramer biosynthetic process, up-regulation of protein homotetramer formation, up-regulation of protein homotetramerization, upregulation of protein homotetramer assembly, upregulation of protein homotetramer biosynthesis, upregulation of protein homotetramer biosynthetic process, upregulation of protein homotetramer formation, upregulation of protein homotetramerization, activation of protein homotetramer assembly, activation of protein homotetramer biosynthesis, activation of protein homotetramer biosynthetic process, activation of protein homotetramer formation, activation of protein homotetramerization Relationships: is a type of GO:0032464; is_a GO:1901092; is a type of GO:1901093; positively regulates protein homotetramerization [GO:0051289] Definition: Any process that activates or increases the frequency, rate or extent of protein homotetramerization.